{
  "gene": "UniProtKB:Q6B0K9",
  "term_id": "GO:0015671",
  "gene_symbol": "HBM",
  "term_label": "oxygen transport",
  "gene_name": "Hemoglobin subunit mu"
}